{
  "gene_name": "UL16-binding protein 1",
  "term_label": "external side of plasma membrane",
  "term_id": "GO:0009897",
  "gene_symbol": "ULBP1",
  "gene": "UniProtKB:Q9BZM6"
}